{
  "gene_name": "Junctional cadherin 5-associated protein",
  "gene_symbol": "JCAD",
  "term_id": "GO:0005912",
  "gene": "UniProtKB:Q9P266",
  "term_label": "adherens junction"
}